{
  "gene": "UniProtKB:O75818",
  "gene_name": "Ribonuclease P protein subunit p40",
  "term_label": "ribonuclease MRP complex",
  "term_id": "GO:0000172",
  "gene_symbol": "RPP40"
}